cellular response to erythropoietin [GO:0036018] (biological process) Relationships: is a type of response to erythropoietin [GO:0036017]; is a type of cellular response to cytokine stimulus [GO:0071345] Sources: GOC:yaf Definition: Any process that results in a change in state or activity of a cell (in terms of movement, secretion, enzyme production, gene expression, etc.) as a result of an erythropoietin stimulus.